{
  "gene": "UniProtKB:P21439",
  "term_id": "GO:0090554",
  "term_label": "phosphatidylcholine floppase activity",
  "gene_name": "Phosphatidylcholine translocator ABCB4",
  "gene_symbol": "ABCB4"
}